{
  "gene_name": "Beclin 1-associated autophagy-related key regulator",
  "gene_symbol": "ATG14",
  "term_id": "GO:0035014",
  "term_label": "phosphatidylinositol 3-kinase regulator activity",
  "gene": "UniProtKB:Q6ZNE5"
}